icosahedral viral capsid, spike [GO:0098029] (cellular component) Definition: A short structure attached to an icosahedral virion capsid, and used for attachment to the host cell. Sources: GOC:bm Relationships: is a type of virion component [GO:0044423]; is part of icosahedral viral capsid [GO:0019030]